{
  "term_id": "GO:0031204",
  "gene_symbol": "SEC61B",
  "gene_name": "Protein transport protein Sec61 subunit beta",
  "gene": "UniProtKB:P60468",
  "term_label": "post-translational protein targeting to membrane, translocation"
}